{
  "gene": "UniProtKB:Q96QT4",
  "gene_name": "Transient receptor potential cation channel subfamily M member 7",
  "term_id": "GO:0005262",
  "gene_symbol": "TRPM7",
  "term_label": "calcium channel activity"
}